{
  "gene_symbol": "STAG1",
  "term_id": "GO:0003682",
  "gene_name": "Cohesin subunit SA-1",
  "term_label": "chromatin binding",
  "gene": "UniProtKB:Q8WVM7"
}